{
  "term_label": "intra-Golgi vesicle-mediated transport",
  "gene_name": "Coatomer subunit gamma-2",
  "gene_symbol": "COPG2",
  "term_id": "GO:0006891",
  "gene": "UniProtKB:Q9UBF2"
}